hypoxanthine biosynthetic process [GO:0046101] (biological process) Definition: The chemical reactions and pathways resulting in the formation of hypoxanthine, 6-hydroxy purine, an intermediate in the degradation of adenylate. Its ribonucleoside is known as inosine and its ribonucleotide as inosinate. Sources: GOC:go_curators Also known as: hypoxanthine anabolism, hypoxanthine biosynthesis, hypoxanthine formation, hypoxanthine synthesis Relationships: is a type of purine nucleobase biosynthetic process [GO:0009113]; is a type of hypoxanthine metabolic process [GO:0046100] Subtypes: GO:0043103